{
  "term_label": "regulation of transcription by RNA polymerase II",
  "term_id": "GO:0006357",
  "gene_name": "Homeobox protein DLX-5",
  "gene_symbol": "DLX5",
  "gene": "UniProtKB:P56178"
}